{
  "gene_symbol": "GLUL",
  "gene": "UniProtKB:P15104",
  "term_label": "glutamine synthetase activity",
  "gene_name": "Glutamine synthetase",
  "term_id": "GO:0004356"
}